pigment catabolic process [GO:0046149] (biological process) Also known as: pigment breakdown, pigment catabolism, pigment degradation Definition: The chemical reactions and pathways resulting in the breakdown of a pigment, any general or particular coloring matter in living organisms, e.g. melanin. Relationships: is a type of GO:0042440 Sources: ISBN:0198506732 Subtypes: chlorophyll catabolic process [GO:0015996], heme catabolic process [GO:0042167], GO:0046150, eye pigment catabolic process [GO:0046151], GO:0046159, anthocyanin-containing compound catabolic process [GO:0046284]